{
  "term_id": "GO:0030956",
  "term_label": "glutamyl-tRNA(Gln) amidotransferase complex",
  "gene_symbol": "QRSL1",
  "gene_name": "Glutamyl-tRNA(Gln) amidotransferase subunit A, mitochondrial",
  "gene": "UniProtKB:Q9H0R6"
}